{
  "term_id": "UNKNOWN:0003",
  "gene": "UniProtKB:P13224",
  "term_label": "Unknown cellular component",
  "gene_symbol": "GP1BB",
  "gene_name": "Platelet glycoprotein Ib beta chain"
}